{
  "gene_symbol": "GPR151",
  "term_id": "GO:0004930",
  "term_label": "G protein-coupled receptor activity",
  "gene": "UniProtKB:Q8TDV0",
  "gene_name": "G-protein coupled receptor 151"
}